{
  "gene": "UniProtKB:A8MTT3",
  "term_label": "Unknown molecular function",
  "gene_symbol": "CEBPZOS",
  "gene_name": "Protein CEBPZOS",
  "term_id": "UNKNOWN:0001"
}